{
  "gene_name": "Interleukin-1 receptor-associated kinase 1-binding protein 1",
  "term_label": "Unknown molecular function",
  "gene": "UniProtKB:Q5VVH5",
  "term_id": "UNKNOWN:0001",
  "gene_symbol": "IRAK1BP1"
}